{
  "gene_symbol": "RNF122",
  "term_label": "Unknown molecular function",
  "gene_name": "RING finger protein 122",
  "term_id": "UNKNOWN:0001",
  "gene": "UniProtKB:Q9H9V4"
}